{
  "term_label": "Unknown biological process",
  "gene_symbol": "SLC49A3",
  "term_id": "UNKNOWN:0002",
  "gene": "UniProtKB:Q6UXD7",
  "gene_name": "Solute carrier family 49 member A3"
}